embryonic heart tube development [GO:0035050] (biological process) Sources: GOC:go_curators Relationships: is a type of tube development [GO:0035295]; is a type of epithelium development [GO:0060429]; is part of heart development [GO:0007507]; is part of embryonic organ development [GO:0048568] Definition: The process whose specific outcome is the progression of the embryonic heart tube over time, from its formation to the mature structure. The heart tube forms as the heart rudiment from the heart field.